pimelyl-[acyl-carrier protein] methyl ester esterase activity [GO:0090499] (molecular function) References: PMID:23045647 Sources: RHEA:42700 Definition: Catalysis of the reaction: 6-carboxyhexanoyl-[ACP] methyl ester + H2O = 6-carboxyhexanoyl-[ACP] + H+ + methanol. Relationships: is_a carboxylic ester hydrolase activity [GO:0052689] Note: Note that while this reaction occurs on a modified protein (acyl-carrier protein), the ACP only acts as a carrier that later releases the end product. Also known as: pimelyl-[acyl-carrier protein] methyl ester hydrolase activity